{
  "gene_name": "Enolase 4",
  "term_label": "glycolytic process",
  "gene_symbol": "ENO4",
  "gene": "UniProtKB:A6NNW6",
  "term_id": "GO:0006096"
}